{
  "term_label": "guanyl-nucleotide exchange factor activity",
  "term_id": "GO:0005085",
  "gene_symbol": "RGL1",
  "gene_name": "Ral guanine nucleotide dissociation stimulator-like 1",
  "gene": "UniProtKB:Q9NZL6"
}